{
  "term_label": "type I interferon receptor binding",
  "term_id": "GO:0005132",
  "gene": "UniProtKB:P05015",
  "gene_symbol": "IFNA16",
  "gene_name": "Interferon alpha-16"
}